{
  "term_label": "cytoplasm",
  "gene_symbol": "RPAP2",
  "gene": "UniProtKB:Q8IXW5",
  "gene_name": "Putative RNA polymerase II subunit B1 CTD phosphatase RPAP2",
  "term_id": "GO:0005737"
}